serine-isocitrate lyase pathway [GO:0019496] (biological process) Relationships: is a type of one-carbon metabolic process [GO:0006730] Sources: ISBN:0387961534 Definition: A one-carbon metabolic process in which acetyl-CoA is produced from formaldehyde and carbon dioxide.